{
  "term_id": "GO:0007167",
  "term_label": "enzyme-linked receptor protein signaling pathway",
  "gene_name": "Connector enhancer of kinase suppressor of ras 2",
  "gene": "UniProtKB:Q8WXI2",
  "gene_symbol": "CNKSR2"
}